{
  "term_label": "Unknown biological process",
  "gene_name": "Bridge-like lipid transfer protein family member 2",
  "term_id": "UNKNOWN:0002",
  "gene": "UniProtKB:Q14667",
  "gene_symbol": "BLTP2"
}